negative regulation of thiamine biosynthetic process [GO:0070624] (BP) Definition: Any process that stops, prevents, or reduces the frequency, rate or extent of the chemical reactions and pathways resulting in the formation of thiamine. Also known as: down regulation of thiamine biosynthetic process, down-regulation of thiamine biosynthetic process, downregulation of thiamine biosynthetic process, negative regulation of thiamin biosynthetic process, negative regulation of thiamine anabolism, negative regulation of thiamine biosynthesis, negative regulation of thiamine formation, negative regulation of thiamine synthesis, inhibition of thiamine biosynthetic process Sources: GOC:mah Relationships: is a type of negative regulation of vitamin metabolic process [GO:0046137]; is a type of regulation of thiamine biosynthetic process [GO:0070623]; is a type of negative regulation of alcohol biosynthetic process [GO:1902931]; RO_0002212 GO:0009228